gamete generation [GO:0007276] (biological process) Relationships: is a type of multicellular organismal reproductive process [GO:0048609]; BFO_0000050 sexual reproduction [GO:0019953] Also known as: gametogenesis Sources: GOC:ems, GOC:mtg_sensu Definition: The generation and maintenance of gametes in a multicellular organism. A gamete is a haploid reproductive cell. Subtypes: female gamete generation [GO:0007292], male gamete generation [GO:0048232]